cobaltochelatase activity [GO:0051116] (MF) Definition: Catalysis of the reaction: ATP + Co(2+) + H2O + hydrogenobyrinate a,c-diamide = ADP + cob(II)yrinate a,c diamide + 4 H+ + phosphate. Also known as: hydrogenobyrinic acid a,c-diamide cobaltochelatase activity, CobNST, CobN-CobST, hydrogenobyrinic-acid-a,c-diamide:cobalt cobalt-ligase (ADP-forming) Relationships: is a type of GO:0051003 Sources: EC:6.6.1.2, RHEA:15341